{
  "term_label": "regulation of store-operated calcium entry",
  "gene_name": "GRAM domain-containing protein 2A",
  "gene": "UniProtKB:Q8IUY3",
  "gene_symbol": "GRAMD2A",
  "term_id": "GO:2001256"
}